cellular response to interleukin-2 [GO:0071352] (BP) Also known as: cellular response to IL-2 Sources: GOC:mah Relationships: is_a response to interleukin-2 [GO:0070669]; is a type of cellular response to cytokine stimulus [GO:0071345] Definition: Any process that results in a change in state or activity of a cell (in terms of movement, secretion, enzyme production, gene expression, etc.) as a result of an interleukin-2 stimulus.